negative regulation of egg-laying behavior [GO:1901045] (biological process) Relationships: is a type of regulation of egg-laying behavior [GO:0046662]; is a type of negative regulation of behavior [GO:0048521]; is a type of negative regulation of reproductive process [GO:2000242]; negatively regulates egg-laying behavior [GO:0018991] Sources: GOC:TermGenie, GOC:kmv Definition: Any process that stops, prevents or reduces the frequency, rate or extent of oviposition. Also known as: down regulation of egg laying, down regulation of egg-laying, down-regulation of egg laying, down-regulation of egg-laying, downregulation of egg laying, downregulation of egg-laying, inhibition of egg laying, inhibition of egg-laying, negative regulation of egg laying, negative regulation of egg-laying, down regulation of oviposition, down-regulation of oviposition, downregulation of oviposition, negative regulation of oviposition, inhibition of oviposition